{
  "term_id": "GO:0005886",
  "gene": "UniProtKB:Q19T08",
  "gene_symbol": "ECSCR",
  "term_label": "plasma membrane",
  "gene_name": "Endothelial cell-specific chemotaxis regulator"
}